epigenetic regulation of gene expression [GO:0040029] (biological process) Also known as: regulation of gene expression, epigenetic Subtypes: GO:0007549, epigenetic programming of gene expression [GO:0043045], GO:0045814, GO:0141137 Relationships: is a type of chromatin remodeling [GO:0006338]; is a type of GO:0010468 References: PMID:10521337, PMID:11498582, PMID:22243696, PMID:34414474 Definition: A process that modulates the frequency, rate or extent of gene expression through chromatin remodeling either by modifying higher order chromatin fiber structure, nucleosomal histones, or cytosine methylation of DNA. Once established, this regulation may be maintained over many cell divisions. It can also be heritable in the absence of the instigating signal.